mandibular condyle articular cartilage development [GO:0061978] (biological process) Definition: The process whose specific outcome is the progression of mandibular joint condyle articular cartilage over time, from its formation to the mature structure. References: PMID:20679519 Relationships: is a type of GO:0061976